methionine-oxo-acid transaminase activity [GO:0010326] (molecular function) Relationships: is a type of transaminase activity [GO:0008483] References: PMID:17056707 Sources: RHEA:31763 Definition: Catalysis of the reaction: a 2-oxocarboxylate + L-methionine = 4-methylsulfanyl-2-oxobutanoate + an L-alpha-amino acid. Subtypes: L-methionine:2-oxoglutarate aminotransferase activity [GO:0080099]